{
  "gene_symbol": "FIGNL2",
  "gene": "UniProtKB:A6NMB9",
  "gene_name": "Fidgetin-like protein 2",
  "term_label": "cytoplasm",
  "term_id": "GO:0005737"
}